{
  "term_label": "double-strand break repair via homologous recombination",
  "gene_symbol": "PALB2",
  "gene_name": "Partner and localizer of BRCA2",
  "term_id": "GO:0000724",
  "gene": "UniProtKB:Q86YC2"
}